{
  "term_id": "GO:0038191",
  "gene_symbol": "SEMA4F",
  "gene_name": "Semaphorin-4F",
  "term_label": "neuropilin binding",
  "gene": "UniProtKB:O95754"
}